colanic acid metabolic process [GO:0046377] (biological process) Definition: The chemical reactions and pathways involving colanic acid, a capsular bacterial polysaccharide composed of glucose, galactose, fucose and glucuronic acid residues. Subtypes: colanic acid biosynthetic process [GO:0009242] References: PMID:35630322 Sources: GOC:ai Also known as: colanic acid metabolism Relationships: is a type of macromolecule metabolic process [GO:0043170]; is a type of GO:1901135